{
  "gene": "UniProtKB:Q9H173",
  "term_id": "GO:0005783",
  "gene_name": "Nucleotide exchange factor SIL1",
  "gene_symbol": "SIL1",
  "term_label": "endoplasmic reticulum"
}